{
  "term_label": "signal sequence binding",
  "term_id": "GO:0005048",
  "gene_symbol": "SEC61A1",
  "gene": "UniProtKB:P61619",
  "gene_name": "Protein transport protein Sec61 subunit alpha isoform 1"
}